establishment of endothelial intestinal barrier [GO:0090557] (biological process) References: PMID:22155109 Sources: GOC:krc Definition: The establishment of a barrier between endothelial cell layers of the intestine to exert specific and selective control over the passage of water and solutes, thus allowing formation and maintenance of compartments that differ in fluid and solute composition. Relationships: is a type of establishment of endothelial barrier [GO:0061028]